{
  "gene": "UniProtKB:Q8NEG7",
  "term_id": "UNKNOWN:0002",
  "gene_name": "Protein DENND6B",
  "term_label": "Unknown biological process",
  "gene_symbol": "DENND6B"
}